response to imidacloprid [GO:1902351] (biological process) Definition: Any process that results in a change in state or activity of a cell or an organism (in terms of movement, secretion, enzyme production, gene expression, etc.) as a result of an imidacloprid stimulus. Relationships: is a type of response to nitrogen compound [GO:1901698] References: PMID:23922869 Sources: GOC:TermGenie, GOC:kmv